{
  "gene_name": "Cytochrome P450 2S1",
  "term_id": "GO:0020037",
  "gene_symbol": "CYP2S1",
  "term_label": "heme binding",
  "gene": "UniProtKB:Q96SQ9"
}